{
  "gene_symbol": "MAST4",
  "term_label": "cytoskeleton organization",
  "gene_name": "Microtubule-associated serine_threonine-protein kinase 4",
  "term_id": "GO:0007010",
  "gene": "UniProtKB:O15021"
}